beta-carotene metabolic process [GO:1901810] (biological process) Also known as: beta-carotene metabolism References: PMID:11387982 Sources: GOC:TermGenie, GOC:yaf, MetaCyc:PWY-5943, UniPathway:UPA00802 Relationships: is a type of GO:0016116; is a type of carotene metabolic process [GO:0016119] Definition: The chemical reactions and pathways involving beta-carotene. Subtypes: beta-carotene catabolic process [GO:1901811], GO:1901812